{
  "gene_symbol": "SSU72L5",
  "term_label": "termination of RNA polymerase II transcription",
  "term_id": "GO:0006369",
  "gene": "UniProtKB:A0A1W2PQ64",
  "gene_name": "RNA polymerase II subunit A C-terminal domain phosphatase SSU72 like protein 5"
}